{
  "term_label": "phosphatidylinositol dephosphorylation",
  "gene": "UniProtKB:Q9NTJ5",
  "term_id": "GO:0046856",
  "gene_name": "Phosphatidylinositol-3-phosphatase SAC1",
  "gene_symbol": "SACM1L"
}